{
  "gene": "UniProtKB:Q9NQZ7",
  "gene_name": "Ectonucleoside triphosphate diphosphohydrolase 7",
  "term_label": "Golgi apparatus",
  "gene_symbol": "ENTPD7",
  "term_id": "GO:0005794"
}